{
  "gene_name": "Testis-specific gene 13 protein",
  "term_label": "Unknown cellular component",
  "gene": "UniProtKB:Q96PP4",
  "gene_symbol": "TSGA13",
  "term_id": "UNKNOWN:0003"
}